{
  "gene_symbol": "SDC2",
  "term_label": "Unknown molecular function",
  "gene_name": "Syndecan-2",
  "term_id": "UNKNOWN:0001",
  "gene": "UniProtKB:P34741"
}